{
  "gene": "UniProtKB:Q9Y5Z9",
  "gene_symbol": "UBIAD1",
  "term_label": "menaquinone biosynthetic process",
  "gene_name": "UbiA prenyltransferase domain-containing protein 1",
  "term_id": "GO:0009234"
}